regulation of antibacterial peptide production [GO:0002786] (biological process) Definition: Any process that modulates the frequency, rate, or extent of antibacterial peptide production. Sources: GOC:add Subtypes: GO:0002787, regulation of antibacterial peptide secretion [GO:0002797], positive regulation of antibacterial peptide production [GO:0002803], GO:0002808 Relationships: is a type of regulation of antimicrobial peptide production [GO:0002784]; regulates antibacterial peptide production [GO:0002778]